axonal transport [GO:0098930] (biological process) Subtypes: anterograde axonal transport [GO:0008089], retrograde axonal transport [GO:0008090], axonal transport of mitochondrion [GO:0019896], axonal transport of messenger ribonucleoprotein complex [GO:0099088] Definition: The directed movement of organelles or molecules along microtubules in axons. Also known as: axon cargo transport, axoplasmic transport Sources: ISBN:0815316194 Relationships: is a type of axo-dendritic transport [GO:0008088]; occurs in GO:0030424